{
  "gene": "UniProtKB:Q9NP64",
  "gene_name": "Zinc finger CCHC domain-containing protein 17",
  "gene_symbol": "ZCCHC17",
  "term_id": "UNKNOWN:0003",
  "term_label": "Unknown cellular component"
}